phosphatidylinositol phosphate phosphatase complex [GO:1904144] (cellular component) Note: An example of this is ACPP in human (P15309) in PMID:12525165 (inferred from physical interaction). Relationships: is a type of phosphatase complex [GO:1903293] Subtypes: PTEN phosphatase complex [GO:1990455] Definition: A protein complex which is capable of phosphatidylinositol phosphate phosphatase activity. References: PMID:12525165 Sources: GOC:TermGenie, GOC:bhm, GO_REF:0000088 Also known as: prostatic acid phosphatase complex